{
  "gene_symbol": "EME2",
  "term_label": "Unknown molecular function",
  "term_id": "UNKNOWN:0001",
  "gene": "UniProtKB:A4GXA9",
  "gene_name": "Probable crossover junction endonuclease EME2"
}